NF-kappaB p50/p65 complex [GO:0035525] (cellular component) References: PMID:20393192, PMID:9299584 Sources: GO:add Note: Note that the p50 subunit is encoded by NFKB1 gene in human and the p65 subunit is encoded by the RELA gene in human. Similar nomenclature is used in other vertebrate species. The p50 subunit has a precursor form p105 in some publications. Also known as: NF-kappa B1/RelA complex, NF-kappa B1/p65 complex, NF-kappa p50/RelA complex, NF-kappa p105/RelA complex, NF-kappa p105/p65 complex Definition: A heterodimer of NF-kappa B p50 and p65 subunits. Relationships: is a type of NF-kappaB complex [GO:0071159]